cysteine-type endopeptidase activity [GO:0004197] (molecular function) Definition: Catalysis of the hydrolysis of internal, alpha-peptide bonds in a polypeptide chain by a mechanism in which the sulfhydryl group of a cysteine residue at the active center acts as a nucleophile. Sources: GOC:mah, https://www.ebi.ac.uk/merops/about/glossary.shtml#CATTYPE, https://www.ebi.ac.uk/merops/about/glossary.shtml#ENDOPEPTIDASE Also known as: thiol endopeptidase activity, caspase activity, lysosomal cysteine-type endopeptidase, metacaspase activity Relationships: is a type of endopeptidase activity [GO:0004175]; is a type of cysteine-type peptidase activity [GO:0008234] Subtypes: GPI-anchor transamidase activity [GO:0003923], calcium-dependent cysteine-type endopeptidase activity [GO:0004198], GO:0070137 Regulation: negatively regulated by cysteine-type endopeptidase inhibitor activity [GO:0004869]; positively regulated by cysteine-type endopeptidase activator activity [GO:0140608]